regulation of calcium ion transmembrane transport via high voltage-gated calcium channel [GO:1902514] (biological process) Also known as: regulation of generation of L-type calcium current Relationships: is a type of regulation of calcium ion transmembrane transport [GO:1903169]; regulates calcium ion transmembrane transport via high voltage-gated calcium channel [GO:0061577] References: PMID:1611048 Sources: GOC:TermGenie, GOC:dph, GOC:pg Definition: Any process that modulates the frequency, rate or extent of generation of calcium ion transmembrane transport via high voltage-gated calcium channel. Subtypes: negative regulation of calcium ion transmembrane transport via high voltage-gated calcium channel [GO:1904878], positive regulation of calcium ion transmembrane transport via high voltage-gated calcium channel [GO:1904879]